{
  "gene_symbol": "MRPS21",
  "term_label": "Unknown biological process",
  "gene_name": "Small ribosomal subunit protein bS21m",
  "gene": "UniProtKB:P82921",
  "term_id": "UNKNOWN:0002"
}